meiotic spindle pole body organization [GO:1990395] (biological process) Sources: GOC:vw Definition: A process that is carried out at the cellular level which results in the assembly, arrangement of constituent parts, or disassembly of the meiotic spindle pole body. Relationships: is a type of GO:0051300; is a type of meiotic cell cycle process [GO:1903046]; is part of meiotic spindle organization [GO:0000212]